negative regulation of mating type switching [GO:0031495] (biological process) Sources: GOC:mah Relationships: is a type of regulation of mating type switching [GO:0031494]; is a type of negative regulation of developmental process [GO:0051093]; is a type of GO:2000242; negatively regulates mating type switching [GO:0007533] Also known as: down regulation of mating type switching, down-regulation of mating type switching, downregulation of mating type switching, inhibition of mating type switching Definition: Any process that stops, prevents, or reduces the frequency, rate or extent of mating type switching.